{
  "gene_name": "Probable G-protein coupled receptor 156",
  "gene": "UniProtKB:Q8NFN8",
  "gene_symbol": "GPR156",
  "term_label": "G protein-coupled receptor heterodimeric complex",
  "term_id": "GO:0038039"
}